{
  "term_id": "GO:0000785",
  "gene_symbol": "TSPYL4",
  "gene_name": "Testis-specific Y-encoded-like protein 4",
  "gene": "UniProtKB:Q9UJ04",
  "term_label": "chromatin"
}